{
  "gene": "UniProtKB:P27482",
  "term_label": "centrosome",
  "gene_name": "Calmodulin-like protein 3",
  "term_id": "GO:0005813",
  "gene_symbol": "CALML3"
}